{
  "term_label": "potassium ion leak channel activity",
  "gene_symbol": "KCNK6",
  "gene": "UniProtKB:Q9Y257",
  "term_id": "GO:0022841",
  "gene_name": "Potassium channel subfamily K member 6"
}